{
  "term_id": "GO:0022625",
  "term_label": "cytosolic large ribosomal subunit",
  "gene_symbol": "RPLP0P6",
  "gene_name": "Putative ribosomal protein uL10-like",
  "gene": "UniProtKB:Q8NHW5"
}